{
  "term_id": "GO:0005634",
  "gene": "UniProtKB:Q13469",
  "gene_name": "Nuclear factor of activated T-cells, cytoplasmic 2",
  "gene_symbol": "NFATC2",
  "term_label": "nucleus"
}